{
  "term_label": "regulation of canonical NF-kappaB signal transduction",
  "gene_symbol": "PPM1A",
  "gene": "UniProtKB:P35813",
  "gene_name": "Protein phosphatase 1A",
  "term_id": "GO:0043122"
}